{
  "term_label": "Unknown biological process",
  "gene_name": "Protein LRATD2",
  "gene": "UniProtKB:Q96KN1",
  "term_id": "UNKNOWN:0002",
  "gene_symbol": "LRATD2"
}